{
  "gene_symbol": "GANAB",
  "term_label": "glucan 1,3-alpha-glucosidase activity",
  "gene_name": "Neutral alpha-glucosidase AB",
  "gene": "UniProtKB:Q14697",
  "term_id": "GO:0033919"
}